{
  "gene": "UniProtKB:Q86WG5",
  "gene_name": "Myotubularin-related protein 13",
  "term_label": "Unknown biological process",
  "term_id": "UNKNOWN:0002",
  "gene_symbol": "SBF2"
}